modulation by host of viral molecular function [GO:0044868] (biological process) Subtypes: modulation by host of viral catalytic activity [GO:0044867], modulation by host of RNA binding by virus [GO:1990968] Relationships: is a type of host-mediated perturbation of viral process [GO:0044788]; RO_0002212 GO:0003674 Definition: A process in which a host organism modulates the frequency, rate or extent of any molecular function being mediated by a virus with which it is infected. Sources: GOC:jl